{
  "term_id": "UNKNOWN:0001",
  "gene": "UniProtKB:Q8N118",
  "gene_name": "Cytochrome P450 4X1",
  "gene_symbol": "CYP4X1",
  "term_label": "Unknown molecular function"
}